{
  "term_id": "GO:0005886",
  "gene_symbol": "OR51M1",
  "term_label": "plasma membrane",
  "gene": "UniProtKB:Q9H341",
  "gene_name": "Olfactory receptor 51M1"
}